{
  "term_id": "GO:0006261",
  "gene": "UniProtKB:P35250",
  "gene_symbol": "RFC2",
  "gene_name": "Replication factor C subunit 2",
  "term_label": "DNA-templated DNA replication"
}